DnaB helicase complex [GO:1990161] (cellular component) References: PMID:17947583 Sources: GOC:bhm Definition: A homohexameric protein complex that possesses DNA helicase activity; functions during DNA replication and repair. Also known as: DnaB hexamer Relationships: is a type of DNA helicase complex [GO:0033202]